{
  "gene_name": "T-cell surface glycoprotein CD1b",
  "gene_symbol": "CD1B",
  "term_label": "extracellular space",
  "term_id": "GO:0005615",
  "gene": "UniProtKB:P29016"
}